{
  "gene": "UniProtKB:P02774",
  "gene_symbol": "GC",
  "term_id": "UNKNOWN:0003",
  "term_label": "Unknown cellular component",
  "gene_name": "Vitamin D-binding protein"
}